{
  "gene_symbol": "TAS2R14",
  "gene": "UniProtKB:Q9NYV8",
  "term_label": "membrane",
  "gene_name": "Taste receptor type 2 member 14",
  "term_id": "GO:0016020"
}